regulation of release of sequestered calcium ion into cytosol by sarcoplasmic reticulum [GO:0010880] (biological process) Subtypes: GO:0010881, regulation of skeletal muscle contraction by regulation of release of sequestered calcium ion [GO:0014809] Relationships: is a type of GO:0051279; regulates release of sequestered calcium ion into cytosol by sarcoplasmic reticulum [GO:0014808] Definition: Any process that modulates the rate, frequency or extent of release of sequestered calcium ion into cytosol by the sarcoplasmic reticulum, the process in which the release of sequestered calcium ion by sarcoplasmic reticulum into cytosol occurs via calcium release channels. Sources: GOC:BHF, GOC:dph, GOC:tb